negative regulation of response to biotic stimulus [GO:0002832] (biological process) Definition: Any process that stops, prevents, or reduces the frequency, rate, or extent of a response to biotic stimulus. Sources: GOC:add Also known as: down regulation of response to biotic stimulus, down-regulation of response to biotic stimulus, downregulation of response to biotic stimulus, inhibition of response to biotic stimulus Note: Note that this term is in the subset of terms that should not be used for direct gene product annotation. Instead, select a child term or, if no appropriate child term exists, please request a new term. Direct annotations to this term may be amended during annotation QC. Relationships: is a type of regulation of response to biotic stimulus [GO:0002831]; is a type of negative regulation of response to stimulus [GO:0048585]; negatively regulates response to biotic stimulus [GO:0009607] Subtypes: GO:0002835, negative regulation of antimicrobial humoral response [GO:0008348], negative regulation of systemic acquired resistance [GO:0010113], negative regulation of lipopolysaccharide-mediated signaling pathway [GO:0031665], negative regulation of innate immune response [GO:0045824], GO:0050687, negative regulation of neutrophil mediated killing of symbiont cell [GO:0070955], negative regulation of defense response to insect [GO:1900366], negative regulation of defense response to bacterium [GO:1900425], negative regulation of filamentous growth of a population of unicellular organisms in response to biotic stimulus [GO:1900444], negative regulation of defense response to oomycetes [GO:1902289], negative regulation of xenophagy [GO:1904416]